{
  "term_id": "GO:0019905",
  "gene_name": "Syntaxin-binding protein 5",
  "gene": "UniProtKB:Q5T5C0",
  "term_label": "syntaxin binding",
  "gene_symbol": "STXBP5"
}